priming of cellular response to stress [GO:0080136] (biological process) Definition: The process that enables cells to respond in a more rapid and robust manner than nonprimed cells to much lower levels of a stimulus indicating the organism is under stress. References: PMID:19318610 Also known as: priming of response to stress, priming of stress response Relationships: is a type of regulation of cellular response to stress [GO:0080135]; is part of cellular response to stress [GO:0033554]